{
  "gene_symbol": "DUT",
  "term_id": "GO:0004170",
  "gene": "UniProtKB:P33316",
  "term_label": "dUTP diphosphatase activity",
  "gene_name": "Deoxyuridine 5'-triphosphate nucleotidohydrolase, mitochondrial"
}